{
  "term_id": "GO:0015254",
  "gene_name": "Aquaporin-10",
  "term_label": "glycerol channel activity",
  "gene": "UniProtKB:Q96PS8",
  "gene_symbol": "AQP10"
}